intracellular protein-containing complex [GO:0140535] (cellular component) Subtypes: ubiquitin ligase complex [GO:0000151], GO:0000502, cytosolic tRNA wobble base thiouridylase complex [GO:0002144], GO:0005835, proteasome core complex [GO:0005839], cAMP-dependent protein kinase complex [GO:0005952], CAAX-protein geranylgeranyltransferase complex [GO:0005953], calcium- and calmodulin-dependent protein kinase complex [GO:0005954], calcineurin complex [GO:0005955], protein kinase CK2 complex [GO:0005956], magnesium-dependent protein serine/threonine phosphatase complex [GO:0005963], exodeoxyribonuclease VII complex [GO:0009318], sulfite reductase complex (NADPH) [GO:0009337], exodeoxyribonuclease V complex [GO:0009338], ATP-independent citrate lyase complex [GO:0009346], ethanolamine ammonia-lyase complex [GO:0009350], aminodeoxychorismate synthase complex [GO:0009356], protein-N(PI)-phosphohistidine-sugar phosphotransferase complex [GO:0009357], enterobactin synthetase complex [GO:0009366], ferredoxin hydrogenase complex [GO:0009375], thioglucosidase complex [GO:0010169], GO:0010170, nitrogenase complex [GO:0016610], aminoacyl-tRNA synthetase multienzyme complex [GO:0017101], protein N-acetylglucosaminyltransferase complex [GO:0017122], GO:0030008, CCR4-NOT complex [GO:0030014], GO:0030015, beta-catenin destruction complex [GO:0030877], RNA polymerase complex [GO:0030880], ADPG pyrophosphorylase complex [GO:0030929], GO:0030956, GO:0031026, BLOC complex [GO:0031082], protein acetyltransferase complex [GO:0031248], ubiquitin conjugating enzyme complex [GO:0031371], invertasome [GO:0031421], mannosyltransferase complex [GO:0031501], GO:0031522, nucleotide-activated protein kinase complex [GO:0031588], guanyl-nucleotide exchange factor complex [GO:0032045], GO:0032144, ribonuclease H2 complex [GO:0032299], CBM complex [GO:0032449], SOD1-calcineurin complex [GO:0032517], Bcl3-Bcl10 complex [GO:0032996], vacuolar transporter chaperone complex [GO:0033254], GO:0033256, elongator holoenzyme complex [GO:0033588], GO:0033593, GO:0033607, RNA cap binding complex [GO:0034518], GCH1 complex [GO:0034615], Gemin3-Gemin4-Gemin5 complex [GO:0034716], Gemin6-Gemin7-unrip complex [GO:0034717], GO:0034741, APC-IQGAP complex [GO:0034743], GO:0034744, APC-IQGAP1-Rac1 complex [GO:0034745], GO:0034746, aryl hydrocarbon receptor complex [GO:0034751], ABIN2-NFKB1-MAP3K8 complex [GO:0034977], Hedgehog signaling complex [GO:0035301], GO:0038201, DNA polymerase complex [GO:0042575], DBIRD complex [GO:0044609], methionine adenosyltransferase complex [GO:0048269], GO:0052718, GO:0070214, GO:0070331, CD20-Lck-Lyn-Fyn complex [GO:0070332], GO:0070419, TACC/TOG complex [GO:0070850], CRD-mediated mRNA stability complex [GO:0070937], G-protein alpha(q)-synembrin complex [GO:0071152], G-protein alpha(o)-synembrin complex [GO:0071153], G-protein alpha(i)1-synembrin complex [GO:0071154], GO:0071155, Cdc42 GTPase complex [GO:0071521], tRNA-splicing ligase complex [GO:0072669], centralspindlin complex [GO:0097149], cytosolic [4Fe-4S] assembly targeting complex [GO:0097361], ciliary transition fiber [GO:0097539], BORC complex [GO:0099078], protein folding chaperone complex [GO:0101031], centriolar subdistal appendage [GO:0120103], ubiquitin activating enzyme complex [GO:0120123], ciliary centrin arm [GO:0120269], FMRP-CYFIP1 complex [GO:0160209], GO:1905348, UBR1-RAD6 ubiquitin ligase complex [GO:1990303], MUB1-RAD6-UBR2 ubiquitin ligase complex [GO:1990304], RAD6-UBR2 ubiquitin ligase complex [GO:1990305], RSP5-BUL ubiquitin ligase complex [GO:1990306], RPB4-RPB7 complex [GO:1990328] Definition: A protein-containing complex located intracellularly. Relationships: is a type of GO:0032991 Sources: GOC:pg